{
  "gene": "UniProtKB:O60678",
  "gene_symbol": "PRMT3",
  "term_id": "GO:0006338",
  "gene_name": "Protein arginine N-methyltransferase 3",
  "term_label": "chromatin remodeling"
}